follicular fluid formation in ovarian follicle antrum [GO:0001548] (biological process) Also known as: ovarian follicle antrum/follicular fluid biosynthesis, ovarian follicle antrum/follicular fluid formation Definition: The menstrual cycle process that results in the formation of one central cavity separating the oocyte/cumulus complex from mural granulosa and theca cells during the various stages of oogenesis. Subtypes: GO:0003003, follicular fluid formation in ovarian follicle antrum involved in distinct antral spaces stage [GO:0003004], follicular fluid formation in ovarian follicle antrum involved in scattered antral spaces stage [GO:0003005] Relationships: is a type of ovulation cycle process [GO:0022602]; is part of antral ovarian follicle growth [GO:0001547] Sources: GOC:dph, GOC:tb, https://www.ncbi.nlm.nih.gov/books/NBK279054/